{
  "gene_name": "Testis-expressed sequence 37 protein",
  "term_label": "cytoplasm",
  "gene_symbol": "TEX37",
  "term_id": "GO:0005737",
  "gene": "UniProtKB:Q96LM6"
}